subsynaptic reticulum [GO:0071212] (cellular component) Definition: An elaborate tubulolamellar membrane system that underlies the postsynaptic cell membrane. References: PMID:1460464, PMID:18171947, PMID:19244343, PMID:7946331 Also known as: SSR Relationships: is_a intracellular membrane-bounded organelle [GO:0043231]; is part of cytoplasm [GO:0005737]; BFO_0000050 type I terminal bouton [GO:0061174]